{
  "term_label": "signaling receptor activity",
  "gene_name": "Nyctalopin",
  "gene": "UniProtKB:Q9GZU5",
  "gene_symbol": "NYX",
  "term_id": "GO:0038023"
}